{
  "gene": "UniProtKB:Q63HK5",
  "term_label": "DNA-binding transcription factor activity, RNA polymerase II-specific",
  "gene_symbol": "TSHZ3",
  "term_id": "GO:0000981",
  "gene_name": "Teashirt homolog 3"
}